circadian behavior [GO:0048512] (BP) Subtypes: eclosion rhythm [GO:0008062], circadian sleep/wake cycle process [GO:0022410], GO:0035648, circadian sleep/wake cycle [GO:0042745], locomotor rhythm [GO:0045475] Definition: The specific behavior of an organism that recurs with a regularity of approximately 24 hours. Sources: GOC:bf, GOC:go_curators, GOC:pr Relationships: is_a rhythmic behavior [GO:0007622]; is a type of GO:0007623 Also known as: circadian rhythm behavior